cerebral cortex tangential migration using cell-axon interactions [GO:0021824] (biological process) Relationships: is a type of GO:0021825 Definition: The movement of cerebral cortex neuronal precursors tangentially through the cortex using interaction of the migrating cells with axons of other neurons. References: PMID:12626695 Sources: GOC:cls, GOC:dgh, GOC:dph, GOC:jid, GO_REF:0000021